{
  "gene_name": "Lysophosphatidylcholine acyltransferase 1",
  "term_id": "GO:0005783",
  "gene_symbol": "LPCAT1",
  "term_label": "endoplasmic reticulum",
  "gene": "UniProtKB:Q8NF37"
}